{
  "term_label": "Unknown cellular component",
  "gene_symbol": "CPED1",
  "term_id": "UNKNOWN:0003",
  "gene_name": "Cadherin-like and PC-esterase domain-containing protein 1",
  "gene": "UniProtKB:A4D0V7"
}